{
  "gene": "UniProtKB:P10721",
  "term_label": "plasma membrane",
  "term_id": "GO:0005886",
  "gene_name": "Mast_stem cell growth factor receptor Kit",
  "gene_symbol": "KIT"
}